{
  "term_label": "creatine kinase activity",
  "gene_name": "Creatine kinase M-type",
  "term_id": "GO:0004111",
  "gene": "UniProtKB:P06732",
  "gene_symbol": "CKM"
}